{
  "term_label": "Unknown biological process",
  "gene_name": "Tigger transposable element-derived protein 6",
  "gene_symbol": "TIGD6",
  "term_id": "UNKNOWN:0002",
  "gene": "UniProtKB:Q17RP2"
}